{
  "gene_name": "Solute carrier family 12 member 6",
  "term_id": "GO:1990573",
  "term_label": "potassium ion import across plasma membrane",
  "gene": "UniProtKB:Q9UHW9",
  "gene_symbol": "SLC12A6"
}